{
  "term_id": "GO:0005634",
  "gene_symbol": "MT1X",
  "gene": "UniProtKB:P80297",
  "term_label": "nucleus",
  "gene_name": "Metallothionein-1X"
}